{
  "gene_name": "Biotin--protein ligase",
  "gene": "UniProtKB:P50747",
  "term_label": "biotin--[biotin carboxyl-carrier protein] ligase activity",
  "gene_symbol": "HLCS",
  "term_id": "GO:0004077"
}